{
  "term_id": "GO:0050815",
  "gene": "UniProtKB:P62258",
  "term_label": "phosphoserine residue binding",
  "gene_symbol": "YWHAE",
  "gene_name": "14-3-3 protein epsilon"
}